{
  "gene": "UniProtKB:Q6NZ36",
  "gene_symbol": "FAAP20",
  "term_id": "GO:0043240",
  "gene_name": "Fanconi anemia core complex-associated protein 20",
  "term_label": "Fanconi anaemia nuclear complex"
}